{
  "gene": "UniProtKB:A0A1B0GX95",
  "gene_name": "T cell receptor beta variable 7-4",
  "term_id": "UNKNOWN:0001",
  "term_label": "Unknown molecular function",
  "gene_symbol": "TRBV7-4"
}